{
  "gene": "UniProtKB:A6NGE7",
  "gene_name": "Putative 2-oxo-4-hydroxy-4-carboxy-5-ureidoimidazoline decarboxylase",
  "term_id": "UNKNOWN:0001",
  "term_label": "Unknown molecular function",
  "gene_symbol": "URAD"
}